{
  "term_label": "defense response to virus",
  "gene_symbol": "ISG15",
  "term_id": "GO:0051607",
  "gene_name": "Ubiquitin-like protein ISG15",
  "gene": "UniProtKB:P05161"
}